{
  "gene_symbol": "P0C880",
  "gene": "UniProtKB:P0C880",
  "term_id": "UNKNOWN:0002",
  "term_label": "Unknown biological process",
  "gene_name": "Putative uncharacterized protein FLJ40606"
}